{
  "term_label": "Unknown molecular function",
  "gene_name": "Urotensin-2",
  "term_id": "UNKNOWN:0001",
  "gene_symbol": "UTS2",
  "gene": "UniProtKB:O95399"
}